negative regulation of sporulation resulting in formation of a cellular spore [GO:0042174] (biological process) Sources: GOC:go_curators Definition: Any process that stops, prevents, or reduces the frequency, rate or extent of sporulation. Relationships: is a type of regulation of sporulation resulting in formation of a cellular spore [GO:0042173]; is a type of negative regulation of sporulation [GO:0043939]; negatively regulates sporulation resulting in formation of a cellular spore [GO:0030435] Subtypes: negative regulation of sexual sporulation resulting in formation of a cellular spore [GO:0043942], negative regulation of asexual sporulation resulting in formation of a cellular spore [GO:0043944] Also known as: down regulation of sporulation, down-regulation of sporulation, downregulation of sporulation, inhibition of sporulation